{
  "gene_name": "Crk-like protein",
  "gene": "UniProtKB:P46109",
  "term_label": "receptor tyrosine kinase binding",
  "term_id": "GO:0030971",
  "gene_symbol": "CRKL"
}